{
  "gene": "UniProtKB:Q14651",
  "gene_symbol": "PLS1",
  "term_label": "actin filament network formation",
  "term_id": "GO:0051639",
  "gene_name": "Plastin-1"
}